NAD+ nucleosidase activity, cyclic ADP-ribose generating [GO:0061809] (molecular function) Also known as: ADP-ribosyl cyclase/cyclic ADP-ribose hydrolase, NAD hydrolase, NAD(+) nucleosidase, NADase, nicotinamide adenine dinucleotide nucleosidase Relationships: is a type of hydrolase activity, hydrolyzing N-glycosyl compounds [GO:0016799] References: PMID:11866528 Sources: EC:3.2.2.6 Definition: Catalysis of the reaction: NAD+ + H2O = ADP-D-ribose + nicotinamide + H+, in a two step reaction: first an ADP-ribosyl cyclase reaction to synthesise cyclic ADP-ribose, followed by a cyclic ADP-ribose hydrolase reaction to generate (linear) ADP-ribose.